regulation of protein activation cascade [GO:2000257] (biological process) Relationships: is a type of regulation of protein maturation [GO:1903317]; RO_0002211 GO:0072376 Sources: GOC:mah Definition: Any process that modulates the frequency, rate or extent of protein activation cascade. Subtypes: GO:0002256, regulation of Toll receptor ligand protein activation cascade [GO:0160033], negative regulation of protein activation cascade [GO:2000258], GO:2000259, regulation of blood coagulation, common pathway [GO:2000260], regulation of blood coagulation, extrinsic pathway [GO:2000263], GO:2000266 Also known as: regulation of protein activation pathway, regulation of protein activitory cascade